circadian sleep/wake cycle, REM sleep [GO:0042747] (biological process) Sources: GOC:jl, ISBN:0395825172 Regulation: RO_0002211 by regulation of circadian sleep/wake cycle, REM sleep [GO:0042320]; negatively regulated by negative regulation of circadian sleep/wake cycle, REM sleep [GO:0042322]; positively regulated by positive regulation of circadian sleep/wake cycle, REM sleep [GO:0046005] Relationships: is a type of circadian sleep/wake cycle process [GO:0022410]; is part of circadian sleep/wake cycle, sleep [GO:0050802] Definition: A stage in the circadian sleep cycle during which dreams occur and the body undergoes marked changes including rapid eye movement, loss of reflexes, and increased pulse rate and brain activity.